{
  "term_id": "GO:0003723",
  "gene_symbol": "RPL22",
  "gene": "UniProtKB:P35268",
  "gene_name": "Large ribosomal subunit protein eL22",
  "term_label": "RNA binding"
}